{
  "gene_symbol": "GUSB",
  "gene_name": "Beta-glucuronidase",
  "term_label": "beta-glucuronidase activity",
  "term_id": "GO:0004566",
  "gene": "UniProtKB:P08236"
}